{
  "gene_symbol": "ULBP3",
  "gene": "UniProtKB:Q9BZM4",
  "term_label": "natural killer cell mediated cytotoxicity",
  "gene_name": "UL16-binding protein 3",
  "term_id": "GO:0042267"
}